{
  "gene": "UniProtKB:A0A804HID5",
  "term_label": "Unknown biological process",
  "gene_symbol": "A0A804HID5",
  "gene_name": "Uncharacterized protein",
  "term_id": "UNKNOWN:0002"
}